{
  "gene": "UniProtKB:Q8NGJ7",
  "term_label": "Unknown biological process",
  "gene_name": "Olfactory receptor 51A2",
  "term_id": "UNKNOWN:0002",
  "gene_symbol": "OR51A2"
}